{
  "term_id": "UNKNOWN:0002",
  "term_label": "Unknown biological process",
  "gene": "UniProtKB:A0A1B0GUI7",
  "gene_symbol": "BRD3OS",
  "gene_name": "Putative uncharacterized protein BRD3OS"
}